{
  "term_label": "Unknown molecular function",
  "gene_symbol": "OBP2A",
  "gene_name": "Odorant-binding protein 2a",
  "gene": "UniProtKB:Q9NY56",
  "term_id": "UNKNOWN:0001"
}